{
  "gene_symbol": "TYK2",
  "gene": "UniProtKB:P29597",
  "term_label": "growth hormone receptor binding",
  "gene_name": "Non-receptor tyrosine-protein kinase TYK2",
  "term_id": "GO:0005131"
}